{
  "term_id": "GO:0005886",
  "term_label": "plasma membrane",
  "gene": "UniProtKB:Q695T7",
  "gene_symbol": "SLC6A19",
  "gene_name": "Sodium-dependent neutral amino acid transporter B(0)AT1"
}